{
  "gene_name": "Baculoviral IAP repeat-containing protein 8",
  "gene": "UniProtKB:Q96P09",
  "term_label": "negative regulation of apoptotic process",
  "term_id": "GO:0043066",
  "gene_symbol": "BIRC8"
}